{
  "gene": "UniProtKB:A8MZ59",
  "term_id": "GO:0006357",
  "term_label": "regulation of transcription by RNA polymerase II",
  "gene_name": "Paired-like homeodomain transcription factor LEUTX",
  "gene_symbol": "LEUTX"
}